{
  "gene_symbol": "SELENOI",
  "gene_name": "Ethanolaminephosphotransferase 1",
  "term_label": "Golgi apparatus",
  "gene": "UniProtKB:Q9C0D9",
  "term_id": "GO:0005794"
}